{
  "term_id": "GO:0046961",
  "gene_name": "V-type proton ATPase subunit d 2",
  "gene": "UniProtKB:Q8N8Y2",
  "gene_symbol": "ATP6V0D2",
  "term_label": "proton-transporting ATPase activity, rotational mechanism"
}